{
  "gene": "UniProtKB:Q5THK1",
  "gene_name": "Protein PRR14L",
  "gene_symbol": "PRR14L",
  "term_id": "UNKNOWN:0001",
  "term_label": "Unknown molecular function"
}